{
  "term_label": "Unknown biological process",
  "gene_symbol": "FNDC7",
  "term_id": "UNKNOWN:0002",
  "gene": "UniProtKB:Q5VTL7",
  "gene_name": "Fibronectin type III domain-containing protein 7"
}